pronephric field specification [GO:0039003] (biological process) Definition: The process in which regions of the embryo are delineated into the area in which the pronephric kidney will develop. Also known as: pronephric kidney field specification Sources: GOC:mtg_kidney_jan10 Relationships: is a type of pattern specification involved in pronephros development [GO:0039017]; is a type of kidney field specification [GO:0072004]